regulation of protein refolding [GO:0061083] (BP) Sources: GOC:dph, GOC:tb Subtypes: negative regulation of protein refolding [GO:0061084], positive regulation of protein refolding [GO:1904592] Definition: Any process that regulates the rate, frequency, or extent of protein refolding. Protein refolding is the process carried out by a cell that restores the biological activity of an unfolded or misfolded protein, using helper proteins such as chaperones. Relationships: is a type of regulation of protein folding [GO:1903332]; RO_0002211 protein refolding [GO:0042026]